beta-caryophyllene catabolic process [GO:1901936] (biological process) References: PMID:22867794 Sources: GOC:TermGenie Definition: The chemical reactions and pathways resulting in the breakdown of beta-caryophyllene. Also known as: beta-caryophyllene breakdown, beta-caryophyllene catabolism, beta-caryophyllene degradation Relationships: is a type of sesquiterpene catabolic process [GO:0051763]